detection of temperature stimulus involved in sensory perception [GO:0050961] (biological process) Definition: The series of events in which a temperature stimulus is received and converted into a molecular signal as part of sensory perception. Sources: GOC:ai, GOC:dos Also known as: sensory detection of temperature stimulus, sensory detection of temperature stimulus during sensory perception, sensory detection of thermal stimulus during sensory perception, sensory perception, sensory detection of temperature stimulus, sensory perception, sensory detection of thermal stimulus, sensory perception, sensory transduction of temperature stimulus, sensory perception, sensory transduction of thermal stimulus, sensory transduction of temperature stimulus, sensory transduction of temperature stimulus during sensory perception, sensory transduction of thermal stimulus during sensory perception, sensory detection of heat stimulus during sensory perception, sensory perception, sensory detection of heat stimulus, sensory perception, sensory transduction of heat stimulus, sensory transduction of heat stimulus during sensory perception Relationships: is a type of detection of temperature stimulus [GO:0016048]; is a type of detection of stimulus involved in sensory perception [GO:0050906]; is part of GO:0050951 Subtypes: detection of temperature stimulus involved in thermoception [GO:0050960], detection of temperature stimulus involved in sensory perception of pain [GO:0050965]